sialate 4-O-acetylesterase activity [GO:0106331] (molecular function) References: PMID:22291594 Sources: RHEA:25564 Relationships: is a type of sialate O-acetylesterase activity [GO:0001681] Definition: Catalysis of the reaction: H2O + N-acetyl-4-O-acetylneuraminate = acetate + H+ + N-acetylneuraminate.